{
  "term_id": "GO:0005737",
  "term_label": "cytoplasm",
  "gene": "UniProtKB:Q12988",
  "gene_name": "Heat shock protein beta-3",
  "gene_symbol": "HSPB3"
}